negative regulation of skeletal muscle tissue regeneration [GO:0043417] (biological process) Sources: GOC:jl Subtypes: negative regulation of skeletal muscle satellite cell activation involved in skeletal muscle regeneration [GO:1901667] Relationships: is a type of GO:0043416; is a type of negative regulation of developmental growth [GO:0048640]; is a type of negative regulation of wound healing [GO:0061045]; negatively regulates skeletal muscle tissue regeneration [GO:0043403] Also known as: down regulation of skeletal muscle regeneration, down-regulation of skeletal muscle regeneration, downregulation of skeletal muscle regeneration, inhibition of skeletal muscle regeneration Definition: Any process that stops, prevents, or reduces the frequency, rate or extent of skeletal muscle regeneration.